{
  "gene": "UniProtKB:Q8IWZ4",
  "term_label": "ubiquitin protein ligase activity",
  "gene_name": "E3 ubiquitin-protein ligase TRIM48",
  "gene_symbol": "TRIM48",
  "term_id": "GO:0061630"
}